{
  "term_label": "regulation of immune response",
  "gene_name": "Interleukin-4",
  "gene_symbol": "IL4",
  "gene": "UniProtKB:P05112",
  "term_id": "GO:0050776"
}